pigment binding [GO:0031409] (molecular function) Definition: Binding to a pigment, a general or particular coloring matter in living organisms, e.g. melanin. Sources: GOC:mah Relationships: is a type of binding [GO:0005488] Subtypes: xanthophyll binding [GO:0051738]